post-embryonic pectoral fin morphogenesis [GO:0035130] (biological process) Sources: GOC:dgh Relationships: is a type of post-embryonic appendage morphogenesis [GO:0035120]; is a type of pectoral fin morphogenesis [GO:0035138] Definition: The process, occurring after embryonic development, by which the anatomical structures of the pectoral fin are generated and organized. Pectoral fins are bilaterally paired fins mounted laterally and located behind the gill covers of fish. These fins are used for lateral mobility and propulsion.